{
  "gene_symbol": "LY6H",
  "term_id": "GO:0005886",
  "gene": "UniProtKB:O94772",
  "term_label": "plasma membrane",
  "gene_name": "Lymphocyte antigen 6H"
}